{
  "term_label": "extrinsic component of cytoplasmic side of plasma membrane",
  "gene_symbol": "PLEKHA4",
  "gene": "UniProtKB:Q9H4M7",
  "term_id": "GO:0031234",
  "gene_name": "Pleckstrin homology domain-containing family A member 4"
}